{
  "gene_name": "Conserved oligomeric Golgi complex subunit 7",
  "term_id": "UNKNOWN:0001",
  "gene": "UniProtKB:P83436",
  "term_label": "Unknown molecular function",
  "gene_symbol": "COG7"
}